{
  "gene_symbol": "TAF8",
  "term_label": "Unknown molecular function",
  "gene": "UniProtKB:Q7Z7C8",
  "gene_name": "Transcription initiation factor TFIID subunit 8",
  "term_id": "UNKNOWN:0001"
}